{
  "gene_name": "Cyclic nucleotide-binding domain-containing protein 1",
  "gene_symbol": "CNBD1",
  "term_label": "Unknown biological process",
  "gene": "UniProtKB:Q8NA66",
  "term_id": "UNKNOWN:0002"
}